{
  "term_id": "GO:0045109",
  "gene_symbol": "KRT85",
  "term_label": "intermediate filament organization",
  "gene_name": "Keratin, type II cuticular Hb5",
  "gene": "UniProtKB:P78386"
}